amino acid transmembrane transport [GO:0003333] (biological process) Definition: The process in which an amino acid is transported across a membrane. Sources: GOC:dph, GOC:tb Also known as: amino acid membrane transport Note: Note that this term is not intended for use in annotating lateral movement within membranes. Relationships: is a type of amino acid transport [GO:0006865]; is a type of GO:0055085 Subtypes: GO:0015810, amino acid export across plasma membrane [GO:0032973], amino acid transmembrane export from vacuole [GO:0032974], amino acid transmembrane import into vacuole [GO:0032975], GO:0034487, proline transmembrane transport [GO:0035524], D-alanine transmembrane transport [GO:0042941], GO:0042942, D-methionine transmembrane transport [GO:0048473], amino acid import across plasma membrane [GO:0089718], ornithine transmembrane import into vacuole [GO:0090455], serine import into mitochondrion [GO:0140300], GO:1902475, GO:1903712, GO:1903713, GO:1903714, glycine import into mitochondrion [GO:1904983], basic amino acid transmembrane transport [GO:1990822] Regulation: regulated by regulation of amino acid transmembrane transport [GO:1903789]